positive regulation of renin secretion into blood stream [GO:1900135] (biological process) Relationships: is a type of positive regulation of protein secretion [GO:0050714]; is a type of regulation of renin secretion into blood stream [GO:1900133]; positively regulates GO:0002001 Sources: GOC:TermGenie Definition: Any process that activates or increases the frequency, rate or extent of renin secretion into blood stream. Also known as: positive regulation of renin release into blood stream, up regulation of renin release into blood stream, up regulation of renin secretion into blood stream, up-regulation of renin release into blood stream, up-regulation of renin secretion into blood stream, upregulation of renin release into blood stream, upregulation of renin secretion into blood stream, activation of renin release into blood stream, activation of renin secretion into blood stream